{
  "term_id": "GO:0048245",
  "term_label": "eosinophil chemotaxis",
  "gene": "UniProtKB:P13500",
  "gene_symbol": "CCL2",
  "gene_name": "C-C motif chemokine 2"
}